{
  "gene_name": "Probable phospholipid-transporting ATPase IM",
  "term_label": "phospholipid translocation",
  "term_id": "GO:0045332",
  "gene": "UniProtKB:Q8TF62",
  "gene_symbol": "ATP8B4"
}